short-chain fatty acyl-CoA oxidase activity [GO:0120522] (molecular function) Note: While there is not universal consensus on the lengths of short-, medium-, long- and very-long-chain fatty acids, the GO uses the definitions in ChEBI (see CHEBI:26666, CHEBI:59554, CHEBI:15904 and CHEBI:27283). Definition: Catalysis of the reaction: a short-chain 2,3-saturated fatty acyl-CoA + O2 = a short-chain (2E)-enoyl-CoA + H2O2. Relationships: is a type of acyl-CoA oxidase activity [GO:0003997] Sources: RHEA:78859